{
  "gene_symbol": "GPR89A",
  "term_label": "voltage-gated monoatomic anion channel activity",
  "gene_name": "Golgi pH regulator A",
  "term_id": "GO:0008308",
  "gene": "UniProtKB:B7ZAQ6"
}